{
  "term_id": "UNKNOWN:0001",
  "term_label": "Unknown molecular function",
  "gene": "UniProtKB:Q93100",
  "gene_symbol": "PHKB",
  "gene_name": "Phosphorylase b kinase regulatory subunit beta"
}